{
  "gene_symbol": "MSANTD5",
  "term_label": "Unknown biological process",
  "term_id": "UNKNOWN:0002",
  "gene": "UniProtKB:A0A3B3IT52",
  "gene_name": "Putative uncharacterized protein MSANTD5"
}